{
  "term_label": "actin filament bundle assembly",
  "term_id": "GO:0051017",
  "gene_symbol": "BAIAP2",
  "gene_name": "Brain-specific angiogenesis inhibitor 1-associated protein 2",
  "gene": "UniProtKB:Q9UQB8"
}